{
  "gene_name": "Mitochondrial outer membrane protein SLC25A46",
  "term_id": "GO:0005741",
  "gene_symbol": "SLC25A46",
  "term_label": "mitochondrial outer membrane",
  "gene": "UniProtKB:Q96AG3"
}